{
  "gene_name": "Calcitonin receptor",
  "gene_symbol": "CALCR",
  "term_id": "GO:0007204",
  "term_label": "positive regulation of cytosolic calcium ion concentration",
  "gene": "UniProtKB:P30988"
}